menthol biosynthetic process [GO:0031525] (biological process) Also known as: menthol anabolism, menthol biosynthesis, menthol formation, menthol synthesis Sources: GOC:mah Relationships: is a type of GO:0016099; is a type of GO:1902653 Definition: The chemical reactions and pathways resulting in the formation of menthol, the monoterpene 2-isopropyl-5-methylcyclohexanol.